{
  "term_label": "DNA-binding transcription factor activity, RNA polymerase II-specific",
  "gene_name": "Basic helix-loop-helix transcription factor scleraxis",
  "gene_symbol": "SCX",
  "term_id": "GO:0000981",
  "gene": "UniProtKB:Q7RTU7"
}